{
  "term_id": "UNKNOWN:0001",
  "gene": "UniProtKB:P28290",
  "gene_name": "Protein ITPRID2",
  "gene_symbol": "ITPRID2",
  "term_label": "Unknown molecular function"
}